{
  "gene": "UniProtKB:P0CB33",
  "term_id": "UNKNOWN:0003",
  "gene_symbol": "ZNF735",
  "term_label": "Unknown cellular component",
  "gene_name": "Putative zinc finger protein 735"
}